{
  "gene_symbol": "OLFM1",
  "gene_name": "Noelin",
  "gene": "UniProtKB:Q99784",
  "term_label": "signal transduction",
  "term_id": "GO:0007165"
}